{
  "term_label": "Unknown cellular component",
  "gene_symbol": "ERVK-6",
  "gene_name": "Endogenous retrovirus group K member 6 Pol protein",
  "gene": "UniProtKB:Q9BXR3",
  "term_id": "UNKNOWN:0003"
}